interleukin-10-mediated signaling pathway [GO:0140105] (biological process) Also known as: IL-10-mediated signaling pathway, interleukin-10-mediated signalling pathway References: PMID:11244051 Relationships: is a type of cytokine-mediated signaling pathway [GO:0019221] Definition: The series of molecular signals initiated by interleukin-10 binding to its receptor on the surface of a target cell, and ending with the regulation of a downstream cellular process, e.g. transcription.